{
  "term_label": "translation",
  "gene_symbol": "RPS5",
  "gene_name": "Small ribosomal subunit protein uS7",
  "gene": "UniProtKB:P46782",
  "term_id": "GO:0006412"
}